{
  "gene_name": "Putative POU domain, class 5, transcription factor 1B",
  "gene_symbol": "POU5F1B",
  "gene": "UniProtKB:Q06416",
  "term_label": "DNA-binding transcription factor activity, RNA polymerase II-specific",
  "term_id": "GO:0000981"
}